secondary plasmodesma [GO:0009551] (cellular component) Definition: A plasmodesma with a branched structure, often with many channels leading into a larger central cavity; found in older tissues and usually derived from preexisting primary plasmodesmata. References: PMID:15012255 Relationships: is a type of plasmodesma [GO:0009506]